helper T cell chemotaxis [GO:0035704] (biological process) Relationships: is a type of T cell chemotaxis [GO:0010818] Also known as: T-helper cell chemotaxis Sources: CL:0000912, GOC:BHF Definition: The directed movement of a helper T cell in response to an external stimulus.